cell proliferation involved in embryonic placenta development [GO:0060722] (biological process) Subtypes: spongiotrophoblast cell proliferation [GO:0060720] Sources: GOC:dph Definition: The multiplication or reproduction of cells, resulting in the expansion of the population in the embryonic placenta. Relationships: is a type of cell population proliferation [GO:0008283]; is part of embryonic placenta development [GO:0001892] Regulation: regulated by regulation of cell proliferation involved in embryonic placenta development [GO:0060723]